{
  "gene": "UniProtKB:A6NJY4",
  "gene_name": "Transmembrane protein 238-like",
  "term_id": "UNKNOWN:0002",
  "gene_symbol": "TMEM238L",
  "term_label": "Unknown biological process"
}